fructuronate reductase activity [GO:0008866] (molecular function) Relationships: is a type of GO:0016616 Sources: EC:1.1.1.57, RHEA:15729 Definition: Catalysis of the reaction: D-mannonate + NAD+ = D-fructuronate + H+ + NADH. Also known as: D-mannonate dehydrogenase activity, D-mannonate oxidoreductase activity, D-mannonate:NAD oxidoreductase activity, D-mannonate:NAD+ 5-oxidoreductase activity, mannonate oxidoreductase activity, mannonic dehydrogenase activity